{
  "term_label": "gap junction channel activity",
  "term_id": "GO:0005243",
  "gene": "UniProtKB:P48165",
  "gene_symbol": "GJA8",
  "gene_name": "Gap junction alpha-8 protein"
}